{
  "gene_name": "Chorionic somatomammotropin hormone 2",
  "term_id": "GO:0005131",
  "gene": "UniProtKB:P0DML3",
  "term_label": "growth hormone receptor binding",
  "gene_symbol": "CSH2"
}